SOCS family protein binding [GO:0097678] (molecular function) References: PMID:23885323, PMID:24705897 Sources: GOC:mr, InterPro:IPR028413 Definition: Binding to a member of the suppressor of cytokine signaling (SOCS) family of proteins. SOCS represent an important mechanism to extinguish cytokine and growth factor receptor signaling. Individual SOCS proteins are typically induced by specific cytokines and growth factors, thereby generating a negative feedback loop. SOCS proteins have important functions in development and homeostasis, and in disease, particularly tumor suppression and anti-inflammatory functions. Also known as: suppressor of cytokine signaling family protein binding Relationships: is a type of protein binding [GO:0005515]